{
  "term_label": "apical plasma membrane",
  "gene": "UniProtKB:P15313",
  "gene_name": "V-type proton ATPase subunit B, kidney isoform",
  "term_id": "GO:0016324",
  "gene_symbol": "ATP6V1B1"
}